{
  "gene_name": "Anosmin-1",
  "gene": "UniProtKB:P23352",
  "term_id": "GO:0030182",
  "term_label": "neuron differentiation",
  "gene_symbol": "ANOS1"
}